{
  "term_id": "GO:0005737",
  "gene_symbol": "ARHGAP8",
  "term_label": "cytoplasm",
  "gene_name": "Rho GTPase-activating protein 8",
  "gene": "UniProtKB:P85298"
}